{
  "term_id": "UNKNOWN:0002",
  "gene_name": "von Willebrand factor A domain-containing protein 3B",
  "gene_symbol": "VWA3B",
  "gene": "UniProtKB:Q502W6",
  "term_label": "Unknown biological process"
}